regulation of protein localization to chromosome, telomeric region [GO:1904814] (biological process) Also known as: regulation of protein localisation to chromosome, telomeric region, regulation of protein localization to telomere Relationships: is a type of regulation of protein localization [GO:0032880]; regulates protein localization to chromosome, telomeric region [GO:0070198] Subtypes: negative regulation of protein localization to chromosome, telomeric region [GO:1904815], positive regulation of protein localization to chromosome, telomeric region [GO:1904816] Definition: Any process that modulates the frequency, rate or extent of protein localization to chromosome, telomeric region. References: PMID:19487455 Sources: GOC:BHF, GOC:BHF_telomere, GOC:TermGenie, GOC:nc, GO_REF:0000058